{
  "gene_name": "Small nuclear ribonucleoprotein Sm D1",
  "gene_symbol": "SNRPD1",
  "term_label": "U1 snRNP",
  "term_id": "GO:0005685",
  "gene": "UniProtKB:P62314"
}